{
  "term_id": "GO:0060271",
  "gene_symbol": "BBS7",
  "gene": "UniProtKB:Q8IWZ6",
  "gene_name": "Bardet-Biedl syndrome 7 protein",
  "term_label": "cilium assembly"
}